{
  "gene_symbol": "CAV2",
  "gene_name": "Caveolin-2",
  "term_id": "GO:0060090",
  "term_label": "molecular adaptor activity",
  "gene": "UniProtKB:P51636"
}